{
  "term_id": "GO:0003682",
  "gene_symbol": "ATXN1L",
  "gene_name": "Ataxin-1-like",
  "gene": "UniProtKB:P0C7T5",
  "term_label": "chromatin binding"
}